{
  "gene_name": "Pre-rRNA-processing protein TSR2 homolog",
  "gene": "UniProtKB:Q969E8",
  "term_id": "GO:0000462",
  "gene_symbol": "TSR2",
  "term_label": "maturation of SSU-rRNA from tricistronic rRNA transcript (SSU-rRNA, 5.8S rRNA, LSU-rRNA)"
}